DNA-7-methyladenine glycosylase activity [GO:0052821] (MF) Definition: Catalysis of the reaction: DNA containing 7-methyladenine + H2O = DNA with abasic site + 7-methyladenine. This reaction is the hydrolysis of DNA by cleavage of the N-C1' glycosidic bond between the damaged DNA 7-methyladenine and the deoxyribose sugar to remove the 7-methyladenine, leaving an abasic site. References: PMID:16468998 Sources: GOC:jl Relationships: is a type of alkylbase DNA N-glycosylase activity [GO:0003905]